{
  "gene_symbol": "SNCAIP",
  "gene": "UniProtKB:Q9Y6H5",
  "term_label": "Unknown cellular component",
  "gene_name": "Synphilin-1",
  "term_id": "UNKNOWN:0003"
}